metula development [GO:0070789] (BP) Also known as: development of primary sterigmata Regulation: regulated by regulation of metula development [GO:0070802]; negatively regulated by negative regulation of metula development [GO:0070803]; positively regulated by GO:0070804 Definition: The process whose specific outcome is the progression of metulae over time, from its formation to the mature structure. Metulae are elongated mononucleate cells that bud from the surface of the conidiophore tip. Relationships: is_a GO:0003006; is a type of cell development [GO:0048468]; is part of GO:0070787 References: PMID:9529886